phosphatidylinositol phospholipase C activity [GO:0120548] (molecular function) Sources: RHEA:43484 Definition: Catalysis of the reaction: a 1,2-diacyl-sn-glycero-3-phospho-(1D-myo-inositol) + H2O = 1D-myo-inositol 1-phosphate + a 1,2-diacyl-sn-glycerol + H+. Relationships: is a type of phospholipase C activity [GO:0004629]